response to fibroblast growth factor [GO:0071774] (biological process) Sources: GOC:mah Relationships: is a type of response to growth factor [GO:0070848] Subtypes: GO:0044344 Also known as: response to FGF stimulus, response to fibroblast growth factor stimulus Definition: Any process that results in a change in state or activity of a cell or an organism (in terms of movement, secretion, enzyme production, gene expression, etc.) as a result of a fibroblast growth factor stimulus.